ent-isokaurene C2-hydroxylase activity [GO:0036201] (molecular function) Sources: EC:1.14.14.76 Definition: Catalysis of the reaction: ent-isokaurene + O2 + NADPH + H+ = ent-2alpha-hydroxyisokaurene + H2O + NADP+. Relationships: is a type of oxidoreductase activity, acting on paired donors, with incorporation or reduction of molecular oxygen, NAD(P)H as one donor, and incorporation of one atom of oxygen [GO:0016709]